{
  "term_id": "UNKNOWN:0002",
  "term_label": "Unknown biological process",
  "gene_name": "WAS_WASL-interacting protein family member 2",
  "gene_symbol": "WIPF2",
  "gene": "UniProtKB:Q8TF74"
}